glutamate 5-kinase activity [GO:0004349] (MF) Sources: EC:2.7.2.11, RHEA:14877 Relationships: is a type of GO:0016774; is a type of GO:0019202 Definition: Catalysis of the reaction: L-glutamate + ATP = L-glutamyl 5-phosphate + ADP + H+. Also known as: ATP-L-glutamate 5-phosphotransferase activity, ATP:L-glutamate 5-phosphotransferase activity, ATP:gamma-L-glutamate phosphotransferase activity, gamma-glutamate kinase activity, gamma-glutamyl kinase activity, glutamate kinase activity